{
  "gene_symbol": "SARG",
  "gene_name": "Specifically androgen-regulated gene protein",
  "gene": "UniProtKB:Q9BW04",
  "term_id": "GO:0005737",
  "term_label": "cytoplasm"
}